complement component C5a signaling pathway [GO:0038178] (biological process) References: PMID:15313431 Sources: GOC:jc, Wikipedia:Complement_component_5a Definition: A G protein-coupled receptor signaling pathway initiated by a C5a component of the complement pathway binding to a complement receptor, and ending with regulation of a downstream cellular process. C5a is a peptide derived from the C5 complement factor. Also known as: complement component C5a-induced signaling pathway Relationships: is a type of complement receptor mediated signaling pathway [GO:0002430]; is a type of G protein-coupled receptor signaling pathway [GO:0007186]